{
  "gene_name": "STE20-related kinase adapter protein alpha",
  "term_label": "protein export from nucleus",
  "term_id": "GO:0006611",
  "gene": "UniProtKB:Q7RTN6",
  "gene_symbol": "STRADA"
}